{
  "gene": "UniProtKB:P49407",
  "gene_name": "Beta-arrestin-1",
  "gene_symbol": "ARRB1",
  "term_id": "GO:0060090",
  "term_label": "molecular adaptor activity"
}